{
  "term_id": "GO:0008543",
  "gene_symbol": "FGF2",
  "term_label": "fibroblast growth factor receptor signaling pathway",
  "gene_name": "Fibroblast growth factor 2",
  "gene": "UniProtKB:P09038"
}